aryl-aldehyde dehydrogenase (NAD+) activity [GO:0019108] (molecular function) Sources: EC:1.2.1.29 Definition: Catalysis of the reaction: an aromatic aldehyde + NAD+ + H2O = an aromatic acid + NADH + H+. Also known as: aryl-aldehyde dehydrogenase (NAD) activity, aryl-aldehyde:NAD+ oxidoreductase activity Relationships: is a type of aldehyde dehydrogenase (NAD+) activity [GO:0004029]